{
  "gene": "UniProtKB:P49789",
  "gene_symbol": "FHIT",
  "gene_name": "Bis(5'-adenosyl)-triphosphatase",
  "term_id": "GO:0031625",
  "term_label": "ubiquitin protein ligase binding"
}